{
  "term_label": "nucleoplasm",
  "gene_name": "MORC family CW-type zinc finger protein 4",
  "gene": "UniProtKB:Q8TE76",
  "term_id": "GO:0005654",
  "gene_symbol": "MORC4"
}